{
  "gene_symbol": "GRAMD1A",
  "gene": "UniProtKB:Q96CP6",
  "gene_name": "Protein Aster-A",
  "term_id": "GO:0015485",
  "term_label": "cholesterol binding"
}